regulation of response to type II interferon [GO:0060330] (BP) Subtypes: negative regulation of response to type II interferon [GO:0060331], positive regulation of response to type II interferon [GO:0060332], regulation of type II interferon-mediated signaling pathway [GO:0060334] Also known as: regulation of response to interferon-gamma, regulation of response to immune interferon, regulation of response to type II IFN, regulation of response to gamma-interferon Relationships: is a type of regulation of innate immune response [GO:0045088]; is a type of regulation of response to cytokine stimulus [GO:0060759]; regulates GO:0034341 Definition: Any process that modulates the rate, frequency or extent of a response to type II interferon (interferon-gamma). Response to interferon gamma is a change in state or activity of a cell or an organism (in terms of movement, secretion, enzyme production, gene expression, etc.) as a result of an interferon-gamma stimulus. Sources: GOC:dph